{
  "gene_name": "Inter-alpha-trypsin inhibitor heavy chain H2",
  "gene": "UniProtKB:P19823",
  "gene_symbol": "ITIH2",
  "term_label": "Unknown cellular component",
  "term_id": "UNKNOWN:0003"
}